{
  "gene": "UniProtKB:Q9BPX3",
  "term_label": "cytoplasm",
  "term_id": "GO:0005737",
  "gene_symbol": "NCAPG",
  "gene_name": "Condensin complex subunit 3"
}